regulation of synapse organization [GO:0050807] (biological process) Relationships: is a type of regulation of cellular component organization [GO:0051128]; is part of regulation of synapse structure or activity [GO:0050803]; regulates GO:0050808 Subtypes: regulation of synapse structural plasticity [GO:0051823], regulation of synapse assembly [GO:0051963], regulation of synapse maturation [GO:0090128], regulation of presynapse organization [GO:0099174], regulation of postsynapse organization [GO:0099175], regulation of synaptic membrane adhesion [GO:0099179], regulation of presynaptic membrane organization [GO:1901629], regulation of neuromuscular junction development [GO:1904396], GO:1905244, regulation of synapse pruning [GO:1905806], negative regulation of synapse organization [GO:1905809] Definition: Any process that modulates the physical form of a synapse, the junction between a neuron and a target (neuron, muscle, or secretory cell). Sources: GOC:ai, GOC:dph, GOC:tb Also known as: regulation of synapse organisation, regulation of synapse structure, regulation of synapse organization and biogenesis